{
  "term_id": "GO:0005891",
  "gene_symbol": "CACHD1",
  "term_label": "voltage-gated calcium channel complex",
  "gene": "UniProtKB:Q5VU97",
  "gene_name": "VWFA and cache domain-containing protein 1"
}